{
  "gene_symbol": "POTEE",
  "gene_name": "POTE ankyrin domain family member E",
  "term_label": "membrane",
  "term_id": "GO:0016020",
  "gene": "UniProtKB:Q6S8J3"
}